{
  "gene_symbol": "GAGE5",
  "gene": "UniProtKB:Q13069",
  "term_id": "UNKNOWN:0003",
  "term_label": "Unknown cellular component",
  "gene_name": "G antigen 5"
}